{
  "gene": "UniProtKB:Q9UNZ2",
  "term_id": "GO:0043161",
  "gene_name": "NSFL1 cofactor p47",
  "term_label": "proteasome-mediated ubiquitin-dependent protein catabolic process",
  "gene_symbol": "NSFL1C"
}